{
  "term_label": "cytoplasm",
  "gene_name": "Kinesin-like protein KIF18A",
  "gene_symbol": "KIF18A",
  "term_id": "GO:0005737",
  "gene": "UniProtKB:Q8NI77"
}